{
  "term_label": "Unknown molecular function",
  "term_id": "UNKNOWN:0001",
  "gene": "UniProtKB:A0A1Y8EKQ5",
  "gene_name": "Immunoglobulin heavy diversity 6-19 (Fragment)",
  "gene_symbol": "IGHD6-19"
}